lactosylceramide biosynthetic process [GO:0001572] (BP) Definition: The chemical reactions and pathways resulting in the formation of lactosylceramides that begins with the synthesis of a disaccharide core 4-Gal-beta-1,4-Glc-ceramide. This core can be further elongated with the sequential addition of various carbohydrate units and is also the precursor for the synthesis of gangliosides, globosides and isoglobosides. Also known as: lacto-series glycosphingolipid biosynthesis, lactosylceramide anabolism, lactosylceramide biosynthesis, lactosylceramide formation, lactosylceramide synthesis Relationships: is a type of GO:0006688; is a type of ceramide biosynthetic process [GO:0046513] References: PMID:35536927